{
  "gene": "UniProtKB:Q13489",
  "gene_symbol": "BIRC3",
  "term_label": "cytoplasm",
  "gene_name": "Baculoviral IAP repeat-containing protein 3",
  "term_id": "GO:0005737"
}